{
  "term_id": "GO:0005085",
  "gene": "UniProtKB:O94827",
  "term_label": "guanyl-nucleotide exchange factor activity",
  "gene_symbol": "PLEKHG5",
  "gene_name": "Pleckstrin homology domain-containing family G member 5"
}